methionine-glyoxylate transaminase activity [GO:0050094] (molecular function) Sources: EC:2.6.1.73, RHEA:22884 Definition: Catalysis of the reaction: L-methionine + glyoxylate = 4-methylthio-2-oxobutanoate + glycine. Also known as: L-methionine:glyoxylate aminotransferase activity, MGAT activity, methionine-glyoxylate aminotransferase activity Relationships: is a type of transaminase activity [GO:0008483]